{
  "term_label": "RNA polymerase II cis-regulatory region sequence-specific DNA binding",
  "gene": "UniProtKB:P17535",
  "term_id": "GO:0000978",
  "gene_name": "Transcription factor JunD",
  "gene_symbol": "JUND"
}